NLRP1 inflammasome complex [GO:0072558] (cellular component) Definition: An inflammasome complex that consists of two components, NLRP1 (NALP1) and caspase-1 or caspase-5. The exact mechanisms of NLRP1 activation remain obscure, but potassium ion efflux appears to be essential. References: PMID:20303873 Sources: GOC:BHF, GOC:add, GOC:vp Relationships: is a type of canonical inflammasome complex [GO:0061702] Also known as: NALP1 inflammasome complex